{
  "gene_name": "Large ribosomal subunit protein eL13",
  "term_id": "GO:0003723",
  "gene_symbol": "RPL13",
  "term_label": "RNA binding",
  "gene": "UniProtKB:P26373"
}